{
  "term_id": "GO:0034220",
  "term_label": "monoatomic ion transmembrane transport",
  "gene": "UniProtKB:Q15822",
  "gene_symbol": "CHRNA2",
  "gene_name": "Neuronal acetylcholine receptor subunit alpha-2"
}